norepinephrine-mediated vasodilation [GO:0003122] (biological process) Definition: A vasodilation process resulting from secretion of norepinephrine into the bloodstream or released by nerve endings. Relationships: is a type of vasodilation [GO:0042311] Sources: GOC:mtg_cardio Also known as: regulation of vasodilation by circulating noradrenaline, regulation of vasodilation by circulating norepinephrine, regulation of vasodilation by neuronal noradrenaline, regulation of vasodilation by neuronal norepinephrine, regulation of vasodilation by noradrenaline, regulation of vasodilation by norepinephrine